{
  "term_id": "UNKNOWN:0003",
  "gene_name": "tRNA (cytosine(34)-C(5))-methyltransferase, mitochondrial",
  "gene": "UniProtKB:Q9H649",
  "gene_symbol": "NSUN3",
  "term_label": "Unknown cellular component"
}